{
  "gene_symbol": "ERCC3",
  "gene": "UniProtKB:P19447",
  "term_id": "GO:0043138",
  "gene_name": "General transcription and DNA repair factor IIH helicase subunit XPB",
  "term_label": "3'-5' DNA helicase activity"
}